{
  "term_id": "GO:0006357",
  "gene": "UniProtKB:Q12947",
  "term_label": "regulation of transcription by RNA polymerase II",
  "gene_symbol": "FOXF2",
  "gene_name": "Forkhead box protein F2"
}